{
  "gene": "UniProtKB:Q9NYG2",
  "term_label": "endoplasmic reticulum",
  "gene_name": "Palmitoyltransferase ZDHHC3",
  "gene_symbol": "ZDHHC3",
  "term_id": "GO:0005783"
}